{
  "gene_symbol": "MVB12A",
  "term_id": "GO:0046755",
  "gene_name": "Multivesicular body subunit 12A",
  "term_label": "viral budding",
  "gene": "UniProtKB:Q96EY5"
}